{
  "term_id": "GO:0000122",
  "gene_symbol": "LDB2",
  "gene_name": "LIM domain-binding protein 2",
  "gene": "UniProtKB:O43679",
  "term_label": "negative regulation of transcription by RNA polymerase II"
}